{
  "term_id": "GO:0005829",
  "gene": "UniProtKB:A5LHX3",
  "gene_symbol": "PSMB11",
  "term_label": "cytosol",
  "gene_name": "Proteasome subunit beta type-11"
}